{
  "gene_name": "Gap junction beta-2 protein",
  "term_id": "GO:0007267",
  "gene": "UniProtKB:P29033",
  "term_label": "cell-cell signaling",
  "gene_symbol": "GJB2"
}